{
  "gene_name": "Mothers against decapentaplegic homolog 4",
  "term_label": "SMAD protein signal transduction",
  "gene_symbol": "SMAD4",
  "term_id": "GO:0060395",
  "gene": "UniProtKB:Q13485"
}